{
  "term_label": "DNA-binding transcription factor activity, RNA polymerase II-specific",
  "gene": "UniProtKB:Q16676",
  "gene_symbol": "FOXD1",
  "term_id": "GO:0000981",
  "gene_name": "Forkhead box protein D1"
}